{
  "term_label": "Unknown biological process",
  "gene": "UniProtKB:Q8N8Q3",
  "gene_symbol": "ENDOV",
  "term_id": "UNKNOWN:0002",
  "gene_name": "Endonuclease V"
}